{
  "gene_name": "Leiomodin-3",
  "gene": "UniProtKB:Q0VAK6",
  "term_label": "tropomyosin binding",
  "term_id": "GO:0005523",
  "gene_symbol": "LMOD3"
}